{
  "term_id": "UNKNOWN:0003",
  "term_label": "Unknown cellular component",
  "gene_symbol": "TCEAL3",
  "gene_name": "Transcription elongation factor A protein-like 3",
  "gene": "UniProtKB:Q969E4"
}